negative regulation of neuroblast migration [GO:0061855] (biological process) Relationships: is a type of negative regulation of cell migration [GO:0030336]; is a type of regulation of neuroblast migration [GO:0061853]; negatively regulates GO:0097402 References: PMID:23149556 Definition: Any process that stops, prevents, or reduces the frequency, rate or extent of neuroblast migration.